type IIb hypersensitivity [GO:0001795] (biological process) Sources: GOC:add, ISBN:0781735149 Note: Note that some type IIa hypersensitivity response (GO:0001794) are referred to simply as type II hypersensitivity in the earlier literature, but are mechanistically distinct from type IIb hypersensitivity. Regulation: regulated by GO:0001799; negatively regulated by negative regulation of type IIb hypersensitivity [GO:0001800]; positively regulated by positive regulation of type IIb hypersensitivity [GO:0001801] Also known as: type V hypersensitivity Definition: An inflammatory response resulting in cell death or dysfunction mediated by the direct binding of antibody to cellular receptors. Relationships: is a type of type II hypersensitivity [GO:0002445]